oxalyl-CoA decarboxylase activity [GO:0008949] (molecular function) Definition: Catalysis of the reaction: H+ + oxalyl-CoA = CO2 + formyl-CoA. Sources: EC:4.1.1.8, RHEA:19333 Also known as: oxalyl coenzyme A decarboxylase activity, oxalyl-CoA carboxy-lyase (formyl-CoA-forming), oxalyl-CoA carboxy-lyase activity Relationships: is a type of carboxy-lyase activity [GO:0016831]